{
  "gene": "UniProtKB:O94956",
  "gene_symbol": "SLCO2B1",
  "term_id": "GO:0015721",
  "gene_name": "Solute carrier organic anion transporter family member 2B1",
  "term_label": "bile acid and bile salt transport"
}